{
  "term_label": "immune receptor activity",
  "gene": "UniProtKB:Q14953",
  "term_id": "GO:0140375",
  "gene_symbol": "KIR2DS5",
  "gene_name": "Killer cell immunoglobulin-like receptor 2DS5"
}